response to magnetism [GO:0071000] (BP) Relationships: is a type of response to abiotic stimulus [GO:0009628] Subtypes: cellular response to magnetism [GO:0071259] Definition: Any process that results in a change in state or activity of a cell or an organism (in terms of movement, secretion, enzyme production, gene expression, etc.) as a result of a magnetic stimulus. Sources: GOC:sl Also known as: response to magnetic stimulus